{
  "gene_symbol": "RPL13",
  "gene": "UniProtKB:P26373",
  "term_label": "cytosolic large ribosomal subunit",
  "gene_name": "Large ribosomal subunit protein eL13",
  "term_id": "GO:0022625"
}